{
  "gene_name": "Taste receptor type 2 member 38",
  "term_label": "membrane",
  "gene_symbol": "TAS2R38",
  "term_id": "GO:0016020",
  "gene": "UniProtKB:P59533"
}